{
  "term_label": "plasma membrane",
  "gene": "UniProtKB:Q8TAV4",
  "term_id": "GO:0005886",
  "gene_symbol": "STOML3",
  "gene_name": "Stomatin-like protein 3"
}